endonucleolytic cleavage of tricistronic rRNA transcript (SSU-rRNA, LSU-rRNA, 5S) [GO:0000449] (biological process) Definition: Endonucleolytic cleavage of a pre-rRNA molecule originally produced as a tricistronic rRNA transcript that contains the Small Subunit (SSU) rRNA, the Large Subunit (LSU) rRNA, and the 5S rRNA, in that order, from 5' to 3' along the primary transcript. For example, primary ribosomal RNA transcripts containing three genes, in this order, are produced in E. coli and other prokaryotic species. Note that the use of the word tricistronic refers only to the number of mature rRNA molecules which will be produced from the primary transcript and ignores tRNAs that may also be present within the primary transcript. Sources: GOC:curators Relationships: is a type of rRNA processing [GO:0006364] Subtypes: endonucleolytic cleavage between SSU-rRNA and LSU-rRNA of tricistronic rRNA transcript (SSU-rRNA, LSU-rRNA, 5S) [GO:0000457], endonucleolytic cleavage between LSU-rRNA and 5S rRNA of tricistronic rRNA transcript (SSU-rRNA, LSU-rRNA, 5S) [GO:0000458]